{
  "gene_symbol": "AASDHPPT",
  "term_label": "cytosol",
  "gene": "UniProtKB:Q9NRN7",
  "gene_name": "L-aminoadipate-semialdehyde dehydrogenase-phosphopantetheinyl transferase",
  "term_id": "GO:0005829"
}